{
  "gene_name": "TATA-box-binding protein-associated factor 11-like protein 11",
  "gene_symbol": "TAF11L11",
  "term_label": "RNA polymerase II general transcription initiation factor activity",
  "term_id": "GO:0016251",
  "gene": "UniProtKB:A0A1W2PQ09"
}